{
  "gene_symbol": "NCF2",
  "term_label": "NADPH oxidase complex",
  "term_id": "GO:0043020",
  "gene": "UniProtKB:P19878",
  "gene_name": "Neutrophil cytosol factor 2"
}